{
  "term_id": "GO:0071013",
  "gene_symbol": "DDX23",
  "gene_name": "Probable ATP-dependent RNA helicase DDX23",
  "term_label": "catalytic step 2 spliceosome",
  "gene": "UniProtKB:Q9BUQ8"
}